{
  "gene_name": "Regulator of telomere elongation helicase 1",
  "gene": "UniProtKB:Q9NZ71",
  "gene_symbol": "RTEL1",
  "term_label": "regulation of double-strand break repair via homologous recombination",
  "term_id": "GO:0010569"
}